regulation of filopodium assembly [GO:0051489] (biological process) Definition: Any process that modulates the frequency, rate or extent of the assembly of a filopodium, a thin, stiff protrusion extended by the leading edge of a motile cell such as a crawling fibroblast or amoeba, or an axonal growth cone. Relationships: is a type of GO:0120032; regulates filopodium assembly [GO:0046847] Sources: GOC:ai, GOC:dph, GOC:tb Also known as: regulation of filopodia biosynthesis, regulation of filopodia formation, regulation of filopodium formation Subtypes: GO:0051490, positive regulation of filopodium assembly [GO:0051491]